{
  "gene_name": "Olfactory receptor 2D3",
  "term_label": "olfactory receptor activity",
  "gene": "UniProtKB:Q8NGH3",
  "term_id": "GO:0004984",
  "gene_symbol": "OR2D3"
}